{
  "gene_symbol": "C1QTNF5",
  "gene": "UniProtKB:Q9BXJ0",
  "term_label": "cell projection",
  "gene_name": "Complement C1q tumor necrosis factor-related protein 5",
  "term_id": "GO:0042995"
}